{
  "gene_name": "Phosphorylase b kinase gamma catalytic chain, skeletal muscle_heart isoform",
  "term_label": "cytoplasm",
  "gene": "UniProtKB:Q16816",
  "gene_symbol": "PHKG1",
  "term_id": "GO:0005737"
}